{
  "term_id": "UNKNOWN:0002",
  "gene": "UniProtKB:G3V211",
  "term_label": "Unknown biological process",
  "gene_symbol": "LINC01619",
  "gene_name": "Uncharacterized protein encoded by LINC01619"
}